{
  "term_id": "GO:0071787",
  "term_label": "endoplasmic reticulum tubular network formation",
  "gene_symbol": "RTN4",
  "gene": "UniProtKB:Q9NQC3",
  "gene_name": "Reticulon-4"
}